{
  "term_label": "zeaxanthin biosynthetic process",
  "gene": "UniProtKB:Q16518",
  "gene_symbol": "RPE65",
  "term_id": "GO:1901827",
  "gene_name": "Retinoid isomerohydrolase"
}